{
  "gene": "UniProtKB:Q9P296",
  "gene_symbol": "C5AR2",
  "term_label": "complement receptor mediated signaling pathway",
  "gene_name": "C5a anaphylatoxin chemotactic receptor 2",
  "term_id": "GO:0002430"
}